{
  "term_label": "Unknown biological process",
  "gene": "UniProtKB:P59539",
  "gene_symbol": "TAS2R45",
  "term_id": "UNKNOWN:0002",
  "gene_name": "Taste receptor type 2 member 45"
}